{
  "gene_name": "GREB1-like protein",
  "term_id": "GO:0002009",
  "gene_symbol": "GREB1L",
  "term_label": "morphogenesis of an epithelium",
  "gene": "UniProtKB:Q9C091"
}